internal protein amino acid acetylation [GO:0006475] (biological process) Subtypes: internal peptidyl-lysine acetylation [GO:0018393] Definition: The addition of an acetyl group to a non-terminal amino acid in a protein. Sources: GOC:mah Relationships: is a type of protein acetylation [GO:0006473]